{
  "term_label": "cytoskeleton-nuclear membrane anchor activity",
  "gene_name": "Nesprin-2",
  "gene_symbol": "SYNE2",
  "gene": "UniProtKB:Q8WXH0",
  "term_id": "GO:0140444"
}